structural constituent of presynapse [GO:0099181] (molecular function) References: PMID:23751498 Sources: GOC:dos Definition: The action of a molecule that contributes to the structural integrity of a presynapse. Subtypes: structural constituent of presynaptic actin cytoskeleton [GO:0098699] Relationships: is a type of structural constituent of synapse [GO:0098918]; is part of presynapse organization [GO:0099172]; occurs in presynapse [GO:0098793]